{
  "gene_symbol": "LBP",
  "gene": "UniProtKB:P18428",
  "gene_name": "Lipopolysaccharide-binding protein",
  "term_id": "GO:0001530",
  "term_label": "lipopolysaccharide binding"
}